regulation of chemokine (C-C motif) ligand 5 production [GO:0071649] (biological process) Also known as: regulation of CCL5 production, regulation of RANTES production, regulation of Regulated upon Activation, Normal T-cell Expressed, and Secreted production Subtypes: negative regulation of chemokine (C-C motif) ligand 5 production [GO:0071650], positive regulation of chemokine (C-C motif) ligand 5 production [GO:0071651] Relationships: is a type of regulation of chemokine production [GO:0032642]; regulates GO:0071609 Definition: Any process that modulates the frequency, rate, or extent of production of chemokine (C-C motif) ligand 5. Sources: GOC:mah